cysteine-type endopeptidase inhibitor activity involved in apoptotic process [GO:0043027] (molecular function) References: PMID:14744432 Sources: GOC:jl, GOC:mtg_apoptosis, Wikipedia:Caspase Relationships: is a type of cysteine-type endopeptidase regulator activity involved in apoptotic process [GO:0043028] Definition: Binds to and stops, prevents or reduces the activity of a cysteine-type endopeptidase involved in the apoptotic process. Also known as: caspase inhibitor activity